2-hydroxy-dATP hydrolase activity [GO:0106378] (molecular function) Definition: Catalysis of the reaction: 2-hydroxy-dATP + H2O = 2-hydroxy-dAMP + H+ + diphosphate. Relationships: is a type of GO:0047429 References: PMID:11139615 Sources: RHEA:31583